{
  "term_id": "GO:0007200",
  "gene_name": "C5a anaphylatoxin chemotactic receptor 2",
  "term_label": "phospholipase C-activating G protein-coupled receptor signaling pathway",
  "gene": "UniProtKB:Q9P296",
  "gene_symbol": "C5AR2"
}